{
  "gene_symbol": "FAM89A",
  "term_id": "UNKNOWN:0001",
  "term_label": "Unknown molecular function",
  "gene": "UniProtKB:Q96GI7",
  "gene_name": "Protein FAM89A"
}